epithelial to mesenchymal transition involved in endocardial cushion formation [GO:0003198] (biological process) Sources: GOC:mtg_heart Relationships: is_a cardiac epithelial to mesenchymal transition [GO:0060317]; is part of endocardial cushion formation [GO:0003272] Definition: A transition where a cardiac epithelial cell loses apical/basolateral polarity, severs intercellular adhesive junctions, degrades basement membrane components and becomes a migratory mesenchymal cell that will contribute to the formation of the endocardial cushion. Regulation: RO_0002211 by GO:1905005; negatively regulated by negative regulation of epithelial to mesenchymal transition involved in endocardial cushion formation [GO:1905006]; positively regulated by positive regulation of epithelial to mesenchymal transition involved in endocardial cushion formation [GO:1905007]